{
  "gene": "UniProtKB:P02750",
  "term_id": "GO:0034713",
  "gene_symbol": "LRG1",
  "term_label": "type I transforming growth factor beta receptor binding",
  "gene_name": "Leucine-rich alpha-2-glycoprotein"
}